lysine N-methyltransferase activity [GO:0016278] (molecular function) Relationships: is a type of GO:0008170; is a type of GO:0008757 Sources: GOC:mah Definition: Catalysis of the transfer of a methyl group from S-adenosyl-L-methionine to the epsilon-amino group of a lysine residue. Subtypes: protein-lysine N-methyltransferase activity [GO:0016279]